peptidyl-cysteine S-nitrosylation [GO:0018119] (biological process) Definition: The covalent addition of a nitric oxide (NO) group to the sulphur (S) atom of a cysteine residue in a protein, to form peptidyl-S-nitrosyl-L-cysteine. Also known as: S-nitrosylation, protein S-nitrosylation Sources: RESID:AA0230 Subtypes: GO:0035606 Regulation: negatively regulated by negative regulation of peptidyl-cysteine S-nitrosylation [GO:1902083]; regulated by regulation of peptidyl-cysteine S-nitrosylation [GO:2000169]; positively regulated by positive regulation of peptidyl-cysteine S-nitrosylation [GO:2000170] Relationships: is a type of GO:0017014; is a type of peptidyl-cysteine modification [GO:0018198]